regulation of protein localization to cell surface [GO:2000008] (biological process) Also known as: regulation of protein localisation at cell surface, regulation of protein localization at cell surface Definition: Any process that modulates the frequency, rate or extent of protein localization to the cell surface. Sources: GOC:obol Relationships: is a type of regulation of protein localization [GO:0032880]; regulates protein localization to cell surface [GO:0034394] Subtypes: GO:2000009, positive regulation of protein localization to cell surface [GO:2000010]